negative regulation of error-prone translesion synthesis [GO:1904332] (biological process) References: PMID:22761594 Sources: GOC:TermGenie, GOC:kmv, GO_REF:0000058 Relationships: is a type of negative regulation of response to stimulus [GO:0048585]; is a type of regulation of error-prone translesion synthesis [GO:1904331]; is a type of negative regulation of DNA biosynthetic process [GO:2000279]; negatively regulates error-prone translesion synthesis [GO:0042276] Definition: Any process that stops, prevents or reduces the frequency, rate or extent of error-prone translesion synthesis. Also known as: down regulation of error-prone translesion synthesis, down regulation of mutagenic PRR, down-regulation of error-prone translesion synthesis, down-regulation of mutagenic PRR, downregulation of error-prone translesion synthesis, downregulation of mutagenic PRR, negative regulation of mutagenic PRR, inhibition of error-prone translesion synthesis, inhibition of mutagenic PRR, down regulation of error-prone postreplication DNA repair, down regulation of mutagenic postreplication DNA repair, down-regulation of error-prone postreplication DNA repair, down-regulation of mutagenic postreplication DNA repair, downregulation of error-prone postreplication DNA repair, downregulation of mutagenic postreplication DNA repair, inhibition of error-prone postreplication DNA repair, inhibition of mutagenic postreplication DNA repair, negative regulation of error-prone postreplication DNA repair, negative regulation of mutagenic postreplication DNA repair